{
  "gene": "UniProtKB:P27361",
  "gene_symbol": "MAPK3",
  "term_label": "intracellular signal transduction",
  "gene_name": "Mitogen-activated protein kinase 3",
  "term_id": "GO:0035556"
}